positive regulation of protein oligomerization [GO:0032461] (biological process) Also known as: up regulation of protein oligomerization, up-regulation of protein oligomerization, upregulation of protein oligomerization, activation of protein oligomerization, stimulation of protein oligomerization, induction of protein oligomerization Relationships: is a type of positive regulation of protein-containing complex assembly [GO:0031334]; is a type of regulation of protein oligomerization [GO:0032459]; positively regulates protein complex oligomerization [GO:0051259] Definition: Any process that activates or increases the frequency, rate or extent of protein oligomerization. Subtypes: positive regulation of protein homooligomerization [GO:0032464], positive regulation of protein tetramerization [GO:1901092] Sources: GOC:mah